{
  "term_id": "UNKNOWN:0002",
  "term_label": "Unknown biological process",
  "gene_symbol": "DEFB119",
  "gene_name": "Beta-defensin 119",
  "gene": "UniProtKB:Q8N690"
}